autocrine signaling [GO:0035425] (biological process) Also known as: autocrine signalling Sources: GOC:bf, ISBN:3527303782 Relationships: is a type of GO:0007267 Definition: Signaling between cells of the same type. The signal produced by the signaling cell binds to a receptor on, and affects a cell of the same type.